cell wall (1->3)-alpha-glucan metabolic process [GO:0070597] (biological process) Definition: The chemical reactions and pathways involving (1->3)-alpha-D-glucans, compounds composed of glucose residues linked by (1->3)-alpha-D-glucosidic bonds, found in the walls of cells. Subtypes: cell wall (1->3)-alpha-glucan biosynthetic process [GO:0070598], fungal-type cell wall (1->3)-alpha-glucan metabolic process [GO:0070599] Also known as: cell wall 1,3-alpha-glucan metabolic process, cell wall 1,3-alpha-glucan metabolism, cell wall alpha-1,3 glucan metabolic process, cell wall alpha-1,3 glucan metabolism Relationships: is a type of cell wall polysaccharide metabolic process [GO:0010383]; is a type of (1->3)-alpha-glucan metabolic process [GO:0070595] Sources: GOC:mah